interleukin-15 receptor binding [GO:0016170] (molecular function) Definition: Binding to an interleukin-15 receptor. Also known as: IL-15, interleukin-15 receptor ligand Relationships: is_a GO:0005126 Sources: GOC:ai